aldonate transmembrane transporter activity [GO:0042879] (molecular function) Subtypes: phosphoglycerate transmembrane transporter activity [GO:0015120], GO:0015128, L-idonate transmembrane transporter activity [GO:0015568], D-galactonate transmembrane transporter activity [GO:0042881], glycerate transmembrane transporter activity [GO:1901974] Definition: Enables the transfer of aldonate from one side of a membrane to the other. Sources: GOC:jl, GOC:mtg_transport, ISBN:0815340729 Relationships: is a type of carboxylic acid transmembrane transporter activity [GO:0046943]; is part of aldonate transmembrane transport [GO:0042873]